{
  "term_id": "UNKNOWN:0003",
  "term_label": "Unknown cellular component",
  "gene_symbol": "FAM199X",
  "gene": "UniProtKB:Q6PEV8",
  "gene_name": "Protein FAM199X"
}